estrogen secretion [GO:0035937] (biological process) Also known as: oestrogen secretion Regulation: regulated by regulation of estrogen secretion [GO:2000861]; negatively regulated by negative regulation of estrogen secretion [GO:2000862]; positively regulated by GO:2000863 Sources: GOC:sl Definition: The regulated release of estrogen into the circulatory system. Estrogen is a steroid hormone that stimulates or controls the development and maintenance of female sex characteristics in mammals. Relationships: is a type of steroid hormone secretion [GO:0035929]